{
  "gene_name": "Palmitoyltransferase ZDHHC21",
  "term_label": "protein targeting to membrane",
  "gene": "UniProtKB:Q8IVQ6",
  "gene_symbol": "ZDHHC21",
  "term_id": "GO:0006612"
}